{
  "term_id": "GO:2000045",
  "term_label": "regulation of G1/S transition of mitotic cell cycle",
  "gene_symbol": "CDKN2C",
  "gene_name": "Cyclin-dependent kinase 4 inhibitor C",
  "gene": "UniProtKB:P42773"
}